{
  "gene_symbol": "OR6F1",
  "gene_name": "Olfactory receptor 6F1",
  "term_label": "Unknown biological process",
  "term_id": "UNKNOWN:0002",
  "gene": "UniProtKB:Q8NGZ6"
}